ABC-type capsular-polysaccharide transporter activity [GO:0015436] (molecular function) Relationships: is a type of GO:0033284; is a type of ABC-type transporter activity [GO:0140359]; is part of capsular polysaccharide transport [GO:0015776] Definition: Enables the transfer of a solute or solutes from one side of a membrane to the other according to the reaction: ATP + H2O + capsular polysaccharide(in) = ADP + phosphate + capsular polysaccharide(out). Sources: EC:7.6.2.12 Also known as: ATP-dependent capsular-polysaccharide transporter activity, capsular-polysaccharide-transporting ATPase activity, capsular-polysaccharide ABC transporter, ATP phosphohydrolase (capsular-polysaccharide-exporting), ATPase-coupled capsular-polysaccharide transporter activity